{
  "gene_symbol": "PHF3",
  "term_label": "Unknown biological process",
  "gene": "UniProtKB:Q92576",
  "gene_name": "PHD finger protein 3",
  "term_id": "UNKNOWN:0002"
}